{
  "term_id": "GO:0043209",
  "term_label": "myelin sheath",
  "gene": "UniProtKB:P0DP25",
  "gene_name": "Calmodulin-3",
  "gene_symbol": "CALM3"
}